{
  "term_label": "nucleus",
  "gene_symbol": "IRAK1",
  "gene": "UniProtKB:P51617",
  "term_id": "GO:0005634",
  "gene_name": "Interleukin-1 receptor-associated kinase 1"
}